{
  "term_label": "sperm capacitation",
  "term_id": "GO:0048240",
  "gene": "UniProtKB:Q96P56",
  "gene_name": "Cation channel sperm-associated protein 2",
  "gene_symbol": "CATSPER2"
}